{
  "term_label": "ubiquitin protein ligase binding",
  "gene_symbol": "DET1",
  "gene_name": "DET1 homolog",
  "term_id": "GO:0031625",
  "gene": "UniProtKB:Q7L5Y6"
}